{
  "term_id": "GO:0045171",
  "gene_name": "Kelch domain-containing protein 8B",
  "gene_symbol": "KLHDC8B",
  "term_label": "intercellular bridge",
  "gene": "UniProtKB:Q8IXV7"
}